{
  "gene_name": "Putative uncharacterized protein TSPEAR-AS2",
  "gene_symbol": "TSPEAR-AS2",
  "term_id": "UNKNOWN:0001",
  "term_label": "Unknown molecular function",
  "gene": "UniProtKB:P59090"
}